{
  "term_label": "glycophagy",
  "gene_symbol": "WIPI2",
  "gene": "UniProtKB:Q9Y4P8",
  "gene_name": "WD repeat domain phosphoinositide-interacting protein 2",
  "term_id": "GO:0061723"
}